{
  "gene_name": "Bcl-2-like protein 10",
  "gene": "UniProtKB:Q9HD36",
  "term_label": "extrinsic apoptotic signaling pathway in absence of ligand",
  "gene_symbol": "BCL2L10",
  "term_id": "GO:0097192"
}